{
  "gene": "UniProtKB:Q8WV92",
  "term_id": "GO:0030496",
  "term_label": "midbody",
  "gene_name": "MIT domain-containing protein 1",
  "gene_symbol": "MITD1"
}